larval midgut cell programmed cell death [GO:0035096] (biological process) Sources: GOC:bf, GOC:mtg_apoptosis Also known as: larval midgut cell death, programmed cell death of larval midgut cells Relationships: is a type of programmed cell death involved in cell development [GO:0010623]; is part of larval midgut histolysis [GO:0035069] Definition: The stage-specific programmed cell death of cells of the larval midgut, during histolysis of the larval organ.